{
  "term_id": "GO:0006508",
  "gene_name": "Calpain-1 catalytic subunit",
  "gene": "UniProtKB:P07384",
  "gene_symbol": "CAPN1",
  "term_label": "proteolysis"
}